{
  "term_label": "DNA-binding transcription factor activity, RNA polymerase II-specific",
  "gene_name": "Zinc finger protein 219",
  "gene": "UniProtKB:Q9P2Y4",
  "gene_symbol": "ZNF219",
  "term_id": "GO:0000981"
}